4-amino-4-deoxy-L-arabinose transferase activity [GO:0103015] (molecular function) Sources: EC:2.4.2.43, GOC:pz Relationships: is a type of pentosyltransferase activity [GO:0016763] Definition: Catalysis of the reaction: (Kdo)2-lipid A + 2 4-amino-4-deoxy-alpha-L-arabinopyranosyl di-trans,poly-cis-undecaprenyl phosphate = (beta-L-Ara4N)2-(KDO)2-lipid A + 2 ditrans,polycis-undecaprenyl phosphate.